cell-cell adhesion in response to extracellular stimulus [GO:0140039] (biological process) Relationships: is a type of cell-cell adhesion [GO:0098609]; is part of cellular response to stimulus [GO:0051716] References: PMID:14996911 Subtypes: GO:0000752, GO:0000758 Definition: The attachment of one cell to another cell via adhesion molecules as a result of an extracellular stimulus.